{
  "gene_name": "ATP-binding cassette sub-family D member 3",
  "gene_symbol": "ABCD3",
  "gene": "UniProtKB:P28288",
  "term_id": "GO:0042760",
  "term_label": "very long-chain fatty acid catabolic process"
}